{
  "gene_symbol": "ARHGDIG",
  "term_id": "GO:0016020",
  "term_label": "membrane",
  "gene": "UniProtKB:Q99819",
  "gene_name": "Rho GDP-dissociation inhibitor 3"
}